{
  "gene_name": "1-acylglycerol-3-phosphate O-acyltransferase PNPLA3",
  "gene_symbol": "PNPLA3",
  "term_label": "triglyceride catabolic process",
  "gene": "UniProtKB:Q9NST1",
  "term_id": "GO:0019433"
}